coronary sinus valve morphogenesis [GO:0003182] (biological process) Definition: The process in which the structure of the coronary sinus valve is generated and organized. Sources: GOC:mtg_heart Relationships: is a type of heart valve morphogenesis [GO:0003179]; is part of GO:0003178